choline-phosphate cytidylyltransferase activity [GO:0004105] (molecular function) Relationships: is a type of GO:0070567; is part of CDP-choline pathway [GO:0006657] Sources: EC:2.7.7.15 Also known as: CTP:choline-phosphate cytidylyltransferase activity, CDP-choline pyrophosphorylase activity, CDP-choline synthetase activity, CTP-phosphocholine cytidylyltransferase activity, CTP:phosphocholine cytidylyltransferase activity, CTP:phosphorylcholine cytidylyltransferase activity, choline phosphate cytidylyltransferase activity, cytidine diphosphocholine pyrophosphorylase activity, phosphocholine cytidylyltransferase activity, phosphorylcholine cytidylyltransferase activity, phosphorylcholine transferase activity, phosphorylcholine:CTP cytidylyltransferase activity Definition: Catalysis of the reaction: CTP + choline phosphate = diphosphate + CDP-choline.